{
  "term_id": "GO:0005891",
  "gene": "UniProtKB:Q15878",
  "gene_symbol": "CACNA1E",
  "term_label": "voltage-gated calcium channel complex",
  "gene_name": "Voltage-dependent R-type calcium channel subunit alpha-1E"
}